{
  "gene_symbol": "FBXW11",
  "term_label": "kinetochore",
  "gene_name": "F-box_WD repeat-containing protein 11",
  "gene": "UniProtKB:Q9UKB1",
  "term_id": "GO:0000776"
}